{
  "term_label": "cellular response to glucocorticoid stimulus",
  "gene": "UniProtKB:P04083",
  "gene_symbol": "ANXA1",
  "term_id": "GO:0071385",
  "gene_name": "Annexin A1"
}